{
  "term_id": "UNKNOWN:0002",
  "gene_symbol": "TEX13C",
  "gene": "UniProtKB:A0A0J9YWL9",
  "gene_name": "Putative testis-expressed protein 13C",
  "term_label": "Unknown biological process"
}